{
  "gene_name": "Vacuolar protein sorting-associated protein 51 homolog",
  "term_label": "GARP complex",
  "term_id": "GO:0000938",
  "gene_symbol": "VPS51",
  "gene": "UniProtKB:Q9UID3"
}